{
  "gene_symbol": "CTSB",
  "gene_name": "Cathepsin B",
  "term_id": "GO:0051603",
  "term_label": "proteolysis involved in protein catabolic process",
  "gene": "UniProtKB:P07858"
}